{
  "gene": "UniProtKB:O14617",
  "term_id": "GO:0030123",
  "gene_name": "AP-3 complex subunit delta-1",
  "gene_symbol": "AP3D1",
  "term_label": "AP-3 adaptor complex"
}